{
  "term_id": "GO:0048384",
  "gene": "UniProtKB:P19793",
  "term_label": "retinoic acid receptor signaling pathway",
  "gene_symbol": "RXRA",
  "gene_name": "Retinoic acid receptor RXR-alpha"
}